regulation of epinephrine secretion [GO:0014060] (BP) Sources: GOC:ef Also known as: regulation of adrenaline secretion Definition: Any process that modulates the frequency, rate or extent of the regulated release of epinephrine. Subtypes: negative regulation of epinephrine secretion [GO:0032811], positive regulation of epinephrine secretion [GO:0032812] Relationships: is a type of regulation of catecholamine secretion [GO:0050433]; RO_0002211 epinephrine secretion [GO:0048242]